{
  "term_label": "negative regulation of necroptotic process",
  "term_id": "GO:0060546",
  "gene_name": "Baculoviral IAP repeat-containing protein 3",
  "gene_symbol": "BIRC3",
  "gene": "UniProtKB:Q13489"
}